{
  "gene": "UniProtKB:O95478",
  "term_id": "UNKNOWN:0001",
  "gene_symbol": "NSA2",
  "term_label": "Unknown molecular function",
  "gene_name": "Ribosome biogenesis protein NSA2 homolog"
}